{
  "gene_symbol": "GOLGA4",
  "term_id": "GO:0031267",
  "gene": "UniProtKB:Q13439",
  "gene_name": "Golgin subfamily A member 4",
  "term_label": "small GTPase binding"
}